{
  "term_label": "axon guidance",
  "gene_symbol": "SEMA3B",
  "term_id": "GO:0007411",
  "gene_name": "Semaphorin-3B",
  "gene": "UniProtKB:Q13214"
}